{
  "term_label": "camera-type eye morphogenesis",
  "term_id": "GO:0048593",
  "gene": "UniProtKB:Q06945",
  "gene_name": "Transcription factor SOX-4",
  "gene_symbol": "SOX4"
}